L-amino acid metabolic process [GO:0170033] (biological process) Relationships: is_a alpha-amino acid metabolic process [GO:1901605] Also known as: L-alpha-amino acid metabolism, L-amino acid metabolism Sources: GOC:edw Subtypes: argininosuccinate metabolic process [GO:0000053], L-histidine metabolic process [GO:0006547], GO:0006551, GO:0006558, L-serine metabolic process [GO:0006563], L-tryptophan metabolic process [GO:0006568], tyrosine metabolic process [GO:0006570], glutamine family amino acid metabolic process [GO:0009064], peptidyl-proline hydroxylation to 3-hydroxy-L-proline [GO:0018400], peptidyl-proline hydroxylation to 4-hydroxy-L-proline [GO:0018401], 'de novo' NAD+ biosynthetic process from L-aspartate [GO:0034628], GO:0042851, L-cysteine metabolic process [GO:0046439], S-adenosylhomocysteine metabolic process [GO:0046498], hypusine metabolic process [GO:0046516], L-asparagine metabolic process [GO:0070982], L-kynurenine metabolic process [GO:0097052], L-amino acid biosynthetic process [GO:0170034], L-amino acid catabolic process [GO:0170035], GO:1903184 Definition: The chemical reactions and pathways involving an L-amino acid.